phosphatidylinositol-3,4,5-trisphosphate 3-phosphatase activity [GO:0016314] (molecular function) Definition: Catalysis of the reaction: phosphatidylinositol-3,4,5-trisphosphate + H2O = phosphatidylinositol-4,5-bisphosphate + phosphate. Relationships: is a type of phosphatidylinositol trisphosphate phosphatase activity [GO:0034594] Sources: EC:3.1.3.67 Also known as: PI(3)P 3-phosphatase activity, PI(3,4,5)P3 3-phosphatase activity, PtdIns(3,4,5)P3 3-phosphatase activity, 1-phosphatidyl-1D-myo-inositol-3,4,5-trisphosphate 3-phosphohydrolase activity, MMAC1, phosphatidylinositol-3,4,5-trisphosphate 3-phosphohydrolase activity